{
  "gene_symbol": "CLCN5",
  "term_id": "UNKNOWN:0002",
  "gene_name": "H(+)_Cl(-) exchange transporter 5",
  "term_label": "Unknown biological process",
  "gene": "UniProtKB:P51795"
}